kidney smooth muscle tissue development [GO:0072194] (biological process) Sources: GOC:mtg_kidney_jan10 Relationships: is a type of smooth muscle tissue development [GO:0048745]; is part of kidney development [GO:0001822] Definition: The process whose specific outcome is the progression of smooth muscle in the kidney over time, from its formation to the mature structure. Subtypes: mesonephric smooth muscle tissue development [GO:0061214], metanephric smooth muscle tissue development [GO:0072208]